phosphoserine-tRNA(Cys) ligase activity [GO:0043816] (molecular function) Also known as: O-phosphoseryl-tRNA(Cys) synthetase activity, phosphoserine--tRNA(Cys) ligase activity, phosphoserine-tRNACys ligase activity, SepRS Relationships: is a type of aminoacyl-tRNA ligase activity [GO:0004812] References: PMID:17110438 Sources: RHEA:25678 Definition: Catalysis of the reaction: tRNA(Cys) + O-phospho-L-serine + ATP = AMP + diphosphate + phosphoseryl-tRNA(Cys).